{
  "term_id": "GO:0000398",
  "term_label": "mRNA splicing, via spliceosome",
  "gene": "UniProtKB:Q6ZP01",
  "gene_symbol": "RBM44",
  "gene_name": "RNA-binding protein 44"
}